cell wall thickening [GO:0052386] (biological process) Relationships: is a type of cell wall modification [GO:0042545] Subtypes: defense response by cell wall thickening [GO:0052482], callose deposition in cell wall [GO:0052543] Sources: GOC:mtg_pamgo_17jul06 Definition: A type of cell wall modification in which the cell wall is reinforced and made thicker.